{
  "term_label": "Unknown molecular function",
  "gene": "UniProtKB:Q96ST2",
  "gene_name": "Protein IWS1 homolog",
  "term_id": "UNKNOWN:0001",
  "gene_symbol": "IWS1"
}